negative regulation of peripheral B cell deletion [GO:0002909] (biological process) Relationships: is a type of negative regulation of peripheral tolerance induction [GO:0002659]; is a type of negative regulation of B cell mediated immunity [GO:0002713]; is a type of negative regulation of B cell deletion [GO:0002868]; is a type of regulation of peripheral B cell deletion [GO:0002908]; negatively regulates peripheral B cell deletion [GO:0002454] Also known as: down regulation of peripheral B cell deletion, down-regulation of peripheral B cell deletion, downregulation of peripheral B cell deletion, inhibition of peripheral B cell deletion Sources: GOC:add Definition: Any process that stops, prevents, or reduces the frequency, rate, or extent of peripheral B cell deletion.